{
  "term_label": "mitochondrion",
  "gene": "UniProtKB:Q9BYD2",
  "term_id": "GO:0005739",
  "gene_symbol": "MRPL9",
  "gene_name": "Large ribosomal subunit protein bL9m"
}